{
  "term_label": "extracellular space",
  "term_id": "GO:0005615",
  "gene": "UniProtKB:P0DUB6",
  "gene_name": "Alpha-amylase 1A",
  "gene_symbol": "AMY1A"
}